{
  "gene": "UniProtKB:P17024",
  "gene_name": "Zinc finger protein 20",
  "term_label": "regulation of transcription by RNA polymerase II",
  "gene_symbol": "ZNF20",
  "term_id": "GO:0006357"
}